{
  "term_id": "UNKNOWN:0001",
  "gene_symbol": "ZMYM2",
  "gene_name": "Zinc finger MYM-type protein 2",
  "gene": "UniProtKB:Q9UBW7",
  "term_label": "Unknown molecular function"
}